germinal vesicle [GO:0042585] (cellular component) Definition: The enlarged, fluid filled nucleus of a primary oocyte, the development of which is suspended in prophase I of the first meiotic division between embryohood and sexual maturity. References: PMID:19019837 Sources: GOC:jl, GOC:mtg_sensu Relationships: is a type of female germ cell nucleus [GO:0001674] Also known as: primary oocyte nucleus